gastric inhibitory polypeptide receptor binding [GO:0031767] (molecular function) Sources: GOC:mah, GOC:nln Definition: Binding to a gastric inhibitory polypeptide receptor. Also known as: gastric inhibitory polypeptide receptor ligand Relationships: is a type of G protein-coupled receptor binding [GO:0001664]